DCT cell development [GO:0072140] (biological process) Relationships: is a type of cell development [GO:0048468]; is part of DCT cell differentiation [GO:0072069] Definition: The process whose specific outcome is the progression of a distal convoluted tubule cell over time, from its formation to the mature structure. Subtypes: metanephric DCT cell development [GO:0072241] Sources: GOC:mtg_kidney_jan10 Also known as: distal convoluted tubule cell development